{
  "term_id": "UNKNOWN:0001",
  "gene_symbol": "FAM228B",
  "term_label": "Unknown molecular function",
  "gene_name": "Protein FAM228B",
  "gene": "UniProtKB:P0C875"
}